icosanoid transport [GO:0071715] (biological process) Sources: GOC:mah Subtypes: prostaglandin transport [GO:0015732], icosanoid secretion [GO:0032309], leukotriene transport [GO:0071716], GO:0071717, sodium-independent icosanoid transport [GO:0071718], arachidonate transport [GO:1903963] Also known as: eicosanoid transport Definition: The directed movement of icosanoids into, out of or within a cell, or between cells, by means of some agent such as a transporter or pore. Icosanoids are unsaturated C20 fatty acids and skeletally related compounds. Relationships: is a type of GO:0046942